amino acid sensor activity [GO:0140785] (molecular function) Definition: Binding to and responding, e.g. by conformational change, to changes in the cellular level of an amino acid. Sources: GOC:pg Subtypes: tyrosine sensor activity [GO:0120285], GO:0120286, glutamine sensor activity [GO:0140786], GO:0160233 Also known as: amino acid sensing activity Relationships: is_a GO:0140299